pyridoxine biosynthetic process [GO:0008615] (biological process) Also known as: pyridoxine anabolism, pyridoxine biosynthesis, pyridoxine formation, pyridoxine synthesis Definition: The chemical reactions and pathways resulting in the formation of pyridoxine, 2-methyl-3-hydroxy-4,5-bis(hydroxymethyl)pyridine, one of the vitamin B6 compounds. Relationships: is a type of pyridoxine metabolic process [GO:0008614]; is a type of vitamin B6 biosynthetic process [GO:0042819] Sources: GOC:ai